aspyridone B catabolic process [GO:1901520] (biological process) Definition: The chemical reactions and pathways resulting in the breakdown of aspyridone B. Also known as: aspyridone B breakdown, aspyridone B catabolism, aspyridone B degradation Sources: GOC:TermGenie, GOC:di Relationships: is a type of polyketide catabolic process [GO:0030640]; is a type of pyridine-containing compound catabolic process [GO:0072526]